{
  "term_label": "nuclear envelope",
  "gene_symbol": "PARP16",
  "gene_name": "Protein mono-ADP-ribosyltransferase PARP16",
  "term_id": "GO:0005635",
  "gene": "UniProtKB:Q8N5Y8"
}